{
  "gene_name": "Regulating synaptic membrane exocytosis protein 1",
  "gene": "UniProtKB:Q86UR5",
  "term_id": "GO:2000300",
  "term_label": "regulation of synaptic vesicle exocytosis",
  "gene_symbol": "RIMS1"
}